{
  "term_label": "RNA binding",
  "gene": "UniProtKB:P55769",
  "gene_symbol": "SNU13",
  "term_id": "GO:0003723",
  "gene_name": "NHP2-like protein 1"
}